contractile actin filament bundle assembly [GO:0030038] (BP) Subtypes: stress fiber assembly [GO:0043149] Sources: GOC:mah, ISBN:0815316194 Relationships: is a type of GO:0051017 Definition: Assembly of actin filament bundles in which the filaments are loosely packed (approximately 30-60 nm apart) and arranged with opposing polarities; the loose packing allows myosin (usually myosin-II) to enter the bundle.